{
  "term_label": "endopeptidase activity",
  "term_id": "GO:0004175",
  "gene": "UniProtKB:O14773",
  "gene_name": "Tripeptidyl-peptidase 1",
  "gene_symbol": "TPP1"
}